{
  "term_id": "UNKNOWN:0002",
  "gene": "UniProtKB:Q04609",
  "gene_name": "Glutamate carboxypeptidase 2",
  "gene_symbol": "FOLH1",
  "term_label": "Unknown biological process"
}